{
  "term_id": "GO:0005381",
  "gene_name": "Natural resistance-associated macrophage protein 1",
  "gene_symbol": "SLC11A1",
  "term_label": "iron ion transmembrane transporter activity",
  "gene": "UniProtKB:P49279"
}